valerena-4,7(11)-diene synthase activity [GO:0102412] (molecular function) Relationships: is a type of carbon-oxygen lyase activity, acting on phosphates [GO:0016838] Sources: EC:4.2.3.139, GOC:pz Definition: Catalysis of the reaction: 2-trans,6-trans-farnesyl diphosphate(3-) = valerena-4,7(11)-diene + diphosphoric acid.